{
  "gene": "UniProtKB:Q14642",
  "gene_name": "Inositol polyphosphate-5-phosphatase A",
  "gene_symbol": "INPP5A",
  "term_label": "Unknown biological process",
  "term_id": "UNKNOWN:0002"
}